{
  "gene_symbol": "MRPL50",
  "term_label": "mitochondrial large ribosomal subunit",
  "gene_name": "Large ribosomal subunit protein mL50",
  "gene": "UniProtKB:Q8N5N7",
  "term_id": "GO:0005762"
}